myofibroblast contraction [GO:1990764] (biological process) Definition: The actin filament-based process in which cytoplasmic actin filaments slide past one another resulting in contraction of a myofibroblast. References: PMID:19239477 Also known as: MF contraction, MFB contraction Relationships: is a type of GO:0070252 Regulation: regulated by regulation of myofibroblast contraction [GO:1904328]; negatively regulated by negative regulation of myofibroblast contraction [GO:1904329]; positively regulated by positive regulation of myofibroblast contraction [GO:1904330]